{
  "term_label": "calcium channel activity",
  "gene": "UniProtKB:Q9BWQ8",
  "term_id": "GO:0005262",
  "gene_name": "Protein lifeguard 2",
  "gene_symbol": "FAIM2"
}